{
  "gene_symbol": "PHOSPHO2",
  "term_label": "Unknown cellular component",
  "term_id": "UNKNOWN:0003",
  "gene_name": "Pyridoxal phosphate phosphatase PHOSPHO2",
  "gene": "UniProtKB:Q8TCD6"
}